{
  "term_label": "transcription corepressor activity",
  "gene_name": "LIM domain-containing protein 1",
  "term_id": "GO:0003714",
  "gene_symbol": "LIMD1",
  "gene": "UniProtKB:Q9UGP4"
}